anterior lateral line neuromast hair cell differentiation [GO:0048903] (biological process) Definition: The process in which a relatively unspecialized cell acquires specialized features of an anterior lateral line neuromast hair cell. Neuromast hair cells are the sensory receptors of the neuromast and are located in a portion of the neuromast called the sensory strip. Each hair cell of the neuromast is morphologically polarized as a result of the relative position of the single kinocilium and the clusters of stereocilia on its apical surface. There are approximately seven hair cells within each neuromast, with each hair cell innervated by afferent and efferent neurons. Relationships: is a type of neuromast hair cell differentiation [GO:0048886]; is part of anterior lateral line neuromast development [GO:0048901] Sources: ISBN:0125296509, ISBN:0387968377